{
  "gene_symbol": "SERTAD3",
  "term_label": "Unknown molecular function",
  "gene": "UniProtKB:Q9UJW9",
  "term_id": "UNKNOWN:0001",
  "gene_name": "SERTA domain-containing protein 3"
}